{
  "gene": "UniProtKB:Q9HCK0",
  "gene_symbol": "ZBTB26",
  "term_label": "regulation of cytokine production",
  "term_id": "GO:0001817",
  "gene_name": "Zinc finger and BTB domain-containing protein 26"
}